{
  "gene": "UniProtKB:Q9HBJ7",
  "term_label": "G1/S transition of mitotic cell cycle",
  "gene_name": "Ubiquitin carboxyl-terminal hydrolase 29",
  "gene_symbol": "USP29",
  "term_id": "GO:0000082"
}